peptidyl-lysine 4-dioxygenase activity [GO:0106156] (molecular function) Relationships: is a type of 2-oxoglutarate-dependent dioxygenase activity [GO:0016706]; is a type of catalytic activity, acting on a protein [GO:0140096] References: PMID:24486019 Sources: GOC:pde, RHEA:57156 Definition: Catalysis of the reaction: protein L-lysine + 2-oxoglutarate + O2 = protein 4-hydroxy-L-lysine + succinate + CO2.